2,3-dihydroxy-2,3-dihydro-phenylpropionate dehydrogenase activity [GO:0018498] (MF) Relationships: is a type of oxidoreductase activity, acting on the CH-CH group of donors, NAD or NADP as acceptor [GO:0016628] Definition: Catalysis of the reaction: 3-(cis-5,6-dihydroxycyclohexa-1,3-dien-1-yl)propanoate + NAD+ = 3-(2,3-dihydroxyphenyl)propanoate + H+ + NADH. Also converts (2E)-3-(cis-5,6-dihydroxycyclohexa-1,3-dien-1-yl)prop-2-enoate to (2E)-3-(2,3-dihydroxyphenyl)prop-2-enoate. Sources: EC:1.3.1.87